{
  "term_id": "UNKNOWN:0001",
  "gene_symbol": "ST7",
  "term_label": "Unknown molecular function",
  "gene_name": "Suppressor of tumorigenicity 7 protein",
  "gene": "UniProtKB:Q9NRC1"
}